regulation of macrophage inflammatory protein-1 gamma production [GO:0071646] (biological process) Definition: Any process that modulates the frequency, rate, or extent of production of macrophage inflammatory protein-1 gamma. Sources: GOC:mah Also known as: regulation of CCL9 production, regulation of MIP-1g production, regulation of chemokine (C-C motif) ligand 9 production Relationships: is a type of regulation of chemokine production [GO:0032642]; RO_0002211 GO:0071607 Subtypes: negative regulation of macrophage inflammatory protein-1 gamma production [GO:0071647], GO:0071648